{
  "term_label": "Unknown molecular function",
  "term_id": "UNKNOWN:0001",
  "gene": "UniProtKB:O95872",
  "gene_symbol": "GPANK1",
  "gene_name": "G patch domain and ankyrin repeat-containing protein 1"
}